{
  "term_label": "olfactory receptor activity",
  "gene": "UniProtKB:Q8NGF8",
  "term_id": "GO:0004984",
  "gene_name": "Olfactory receptor 4B1",
  "gene_symbol": "OR4B1"
}